{
  "gene_name": "Protein Wnt-8a",
  "term_id": "GO:0005615",
  "gene": "UniProtKB:Q9H1J5",
  "term_label": "extracellular space",
  "gene_symbol": "WNT8A"
}